{
  "gene": "UniProtKB:P04080",
  "term_label": "Unknown biological process",
  "gene_name": "Cystatin-B",
  "gene_symbol": "CSTB",
  "term_id": "UNKNOWN:0002"
}